ATPase-coupled intramembrane lipid transporter activity [GO:0140326] (MF) Definition: Catalysis of the movement of lipids from one membrane leaflet to the other, driven by ATP hydrolysis. This includes flippases and floppases. Relationships: is_a intramembrane lipid transporter activity [GO:0140303]; is a type of ATP-dependent activity [GO:0140657] Subtypes: flippase activity [GO:0140327], floppase activity [GO:0140328] Also known as: phospholipid flippase activity, ATPase-coupled phospholipid transporter activity, ATPase-dependent phospholipid transporter activity, aminophospholipid-transporting ATPase, phospholipid translocating ATPase activity, phospholipid-translocating ATPase activity, phospholipid-transporting ATPase activity References: PMID:16828084